nuclear exosome focus [GO:1990251] (cellular component) References: PMID:16823445, PMID:23980030, PMID:32012158 Sources: GOC:al, GOC:vw Definition: An nuclear body involved in nuclear mRNA surveilllance. Contains at least Mmi1, or an ortholog of it, and the nuclear exosome. Relationships: is a type of nuclear body [GO:0016604]; has part nuclear exosome (RNase complex) [GO:0000176] Also known as: Mmi1 nuclear focus, nuclear body